{
  "term_label": "DNA-binding transcription factor activity, RNA polymerase II-specific",
  "gene_name": "Netrin-1",
  "term_id": "GO:0000981",
  "gene_symbol": "NTN1",
  "gene": "UniProtKB:O95631"
}